{
  "gene_name": "Myosin-7",
  "gene": "UniProtKB:P12883",
  "term_id": "GO:0005737",
  "gene_symbol": "MYH7",
  "term_label": "cytoplasm"
}